{
  "gene": "UniProtKB:P48736",
  "term_label": "cytoplasm",
  "term_id": "GO:0005737",
  "gene_symbol": "PIK3CG",
  "gene_name": "Phosphatidylinositol 4,5-bisphosphate 3-kinase catalytic subunit gamma isoform"
}